chemokine (C-C motif) ligand 2 binding [GO:0035715] (molecular function) Sources: GOC:BHF Also known as: CCL2 binding Relationships: is a type of C-C chemokine binding [GO:0019957] Definition: Binding to chemokine (C-C motif) ligand 2.